{
  "term_id": "GO:0007015",
  "gene": "UniProtKB:Q92974",
  "gene_name": "Rho guanine nucleotide exchange factor 2",
  "gene_symbol": "ARHGEF2",
  "term_label": "actin filament organization"
}